{
  "term_id": "UNKNOWN:0001",
  "gene_symbol": "CDHR2",
  "gene_name": "Cadherin-related family member 2",
  "term_label": "Unknown molecular function",
  "gene": "UniProtKB:Q9BYE9"
}